cellular response to menaquinone [GO:0071308] (biological process) Definition: Any process that results in a change in state or activity of a cell (in terms of movement, secretion, enzyme production, gene expression, etc.) as a result of a menaquinone (vitamin K2) stimulus. Sources: GOC:mah Also known as: cellular response to menatetrenone, cellular response to vitamin K2 Relationships: is a type of GO:0032572; is a type of cellular response to vitamin K [GO:0071307]